5'-3' DNA/RNA helicase activity [GO:0033678] (molecular function) Definition: Unwinding of a DNA/RNA duplex in the 5' to 3' direction, driven by ATP hydrolysis. Sources: GOC:mah Also known as: 5' to 3' DNA/RNA helicase activity, ATP-dependent 5' to 3' DNA/RNA helicase activity, ATP-dependent 5'-3' DNA/RNA helicase activity Relationships: is a type of GO:0033677